{
  "gene": "UniProtKB:Q86U28",
  "gene_name": "Iron-sulfur cluster assembly 2 homolog, mitochondrial",
  "term_id": "GO:0005506",
  "term_label": "iron ion binding",
  "gene_symbol": "ISCA2"
}